{
  "gene_symbol": "C8orf34",
  "gene_name": "Uncharacterized protein C8orf34",
  "term_id": "UNKNOWN:0001",
  "term_label": "Unknown molecular function",
  "gene": "UniProtKB:Q49A92"
}